negative regulation of raffinose biosynthetic process [GO:1900092] (biological process) Relationships: is a type of negative regulation of biosynthetic process [GO:0009890]; is a type of negative regulation of carbohydrate metabolic process [GO:0045912]; is_a GO:1900091; negatively regulates raffinose biosynthetic process [GO:0033529] Also known as: down regulation of raffinose anabolism, down regulation of raffinose biosynthesis, down regulation of raffinose biosynthetic process, down regulation of raffinose formation, down regulation of raffinose synthesis, down-regulation of raffinose anabolism, down-regulation of raffinose biosynthesis, down-regulation of raffinose biosynthetic process, down-regulation of raffinose formation, down-regulation of raffinose synthesis, downregulation of raffinose anabolism, downregulation of raffinose biosynthesis, downregulation of raffinose biosynthetic process, downregulation of raffinose formation, downregulation of raffinose synthesis, inhibition of raffinose anabolism, inhibition of raffinose biosynthesis, inhibition of raffinose formation, inhibition of raffinose synthesis, negative regulation of raffinose anabolism, negative regulation of raffinose biosynthesis, negative regulation of raffinose formation, negative regulation of raffinose synthesis, inhibition of raffinose biosynthetic process Definition: Any process that stops, prevents or reduces the frequency, rate or extent of raffinose biosynthetic process. References: PMID:22307851 Sources: GOC:TermGenie